protein-malonyllysine demalonylase activity [GO:0036054] (molecular function) Definition: Catalysis of the reaction: N(6)-malonyl-L-lysyl-[protein] + NAD+ + H2O = 2''-O-malonyl-ADP-D-ribose + nicotinamide + L-lysyl-[protein]. Relationships: is a type of GO:0016811; is a type of GO:0140096 Also known as: peptidyl-malonyllysine demalonylase activity, protein lysine demalonylation activity, protein malonyl lysine demalonylation activity References: PMID:21908771, PMID:22076378 Sources: RHEA:47672